{
  "term_id": "GO:0004984",
  "gene_name": "Olfactory receptor 6T1",
  "gene_symbol": "OR6T1",
  "gene": "UniProtKB:Q8NGN1",
  "term_label": "olfactory receptor activity"
}